hexokinase-independent signaling [GO:0009748] (biological process) Sources: GOC:mah, GOC:sm Relationships: is a type of hexose mediated signaling [GO:0009757] Definition: The series of molecular signals mediated by hexose and independent of hexokinase. Also known as: hexokinase-independent signalling